regulation of retinal cone cell fate commitment [GO:0060222] (biological process) Relationships: is a type of regulation of cell fate commitment [GO:0010453]; regulates retinal cone cell fate commitment [GO:0046551] Sources: GOC:dph Subtypes: regulation of retinal cone cell fate specification [GO:0042673], negative regulation of retinal cone cell fate commitment [GO:0060226] Definition: Any process that modulates the process in which a cell becomes committed to a retinal cone cell fate. Retinal cone cell fate commitment is the process in which the developmental fate of a cell becomes restricted such that it will develop into a retinal cone cell.